{
  "term_id": "GO:0005634",
  "gene": "UniProtKB:Q9ULC6",
  "term_label": "nucleus",
  "gene_name": "Protein-arginine deiminase type-1",
  "gene_symbol": "PADI1"
}